(2E)-enoyl-CoA hydratase activity [GO:0080023] (molecular function) Also known as: (3R)-3-hydroxyacyl-CoA dehydratase activity, 3R-hydroxyacyl-CoA dehydratase activity Definition: Catalysis of the reaction: a (3R)-3-hydroxyacyl-CoA = a (2E)-enoyl-CoA + H2O. Relationships: is a type of 3-hydroxyacyl-CoA dehydratase activity [GO:0018812] Subtypes: very-long-chain (3R)-3-hydroxyacyl-CoA dehydratase activity [GO:0102158] References: PMID:16982622 Sources: RHEA:26526